{
  "term_id": "GO:0034134",
  "term_label": "toll-like receptor 2 signaling pathway",
  "gene": "UniProtKB:Q8NFZ5",
  "gene_symbol": "TNIP2",
  "gene_name": "TNFAIP3-interacting protein 2"
}